{
  "term_label": "Golgi apparatus",
  "term_id": "GO:0005794",
  "gene_name": "Microsomal triglyceride transfer protein large subunit",
  "gene": "UniProtKB:P55157",
  "gene_symbol": "MTTP"
}